{
  "term_label": "transcription regulator complex",
  "term_id": "GO:0005667",
  "gene_name": "Dachshund homolog 2",
  "gene": "UniProtKB:Q96NX9",
  "gene_symbol": "DACH2"
}